{
  "term_label": "cytoplasm",
  "gene_symbol": "CDC42EP2",
  "gene_name": "Cdc42 effector protein 2",
  "gene": "UniProtKB:O14613",
  "term_id": "GO:0005737"
}